response to bacterial lipoprotein [GO:0032493] (biological process) References: PMID:12077222 Sources: GOC:add Relationships: is a type of response to molecule of bacterial origin [GO:0002237] Definition: Any process that results in a change in state or activity of an organism (in terms of movement, secretion, enzyme production, gene expression, etc.) as a result of a bacterial lipoprotein stimulus. Subtypes: detection of bacterial lipoprotein [GO:0042494], response to bacterial lipopeptide [GO:0070339], GO:0071220